{
  "term_label": "cytoplasm",
  "gene_symbol": "TRIM9",
  "gene": "UniProtKB:Q9C026",
  "gene_name": "E3 ubiquitin-protein ligase TRIM9",
  "term_id": "GO:0005737"
}